{
  "term_label": "actin cytoskeleton organization",
  "term_id": "GO:0030036",
  "gene": "UniProtKB:A8MU46",
  "gene_name": "Smoothelin-like protein 1",
  "gene_symbol": "SMTNL1"
}